O-succinylbenzoate synthase activity [GO:0043748] (molecular function) Definition: Catalysis of the reaction: 2-succinylbenzoate + H2O = 2-succinyl-6-hydroxy-2,4-cyclohexadiene-1-carboxylate. References: PMID:8335646 Relationships: is a type of hydro-lyase activity [GO:0016836]